{
  "gene": "UniProtKB:P02538",
  "gene_name": "Keratin, type II cytoskeletal 6A",
  "term_label": "intermediate filament organization",
  "gene_symbol": "KRT6A",
  "term_id": "GO:0045109"
}